{
  "gene_name": "Fibroblast growth factor receptor 1",
  "gene": "UniProtKB:P11362",
  "term_label": "plasma membrane",
  "gene_symbol": "FGFR1",
  "term_id": "GO:0005886"
}